spindle pole body-led chromosome movement during mitotic interphase [GO:0140405] (biological process) Definition: A microtubule-based process in which chromosomes migrate as a result of rapid spindle pole body (SPB) and centrosome oscillations during mitotic interphase. References: PMID:31483748 Relationships: is a type of microtubule-based movement [GO:0007018]; is_a chromosome localization [GO:0050000]; happens during mitotic interphase [GO:0051329]